{
  "gene_name": "StAR-related lipid transfer protein 7, mitochondrial",
  "term_id": "UNKNOWN:0001",
  "gene_symbol": "STARD7",
  "term_label": "Unknown molecular function",
  "gene": "UniProtKB:Q9NQZ5"
}